{
  "gene_name": "Telomeric repeat-binding factor 2",
  "gene": "UniProtKB:Q15554",
  "term_label": "negative regulation of telomeric D-loop disassembly",
  "gene_symbol": "TERF2",
  "term_id": "GO:1905839"
}